regulation of macrophage colony-stimulating factor production [GO:1901256] (biological process) Subtypes: regulation of granulocyte colony-stimulating factor production [GO:0071655], GO:1901257, positive regulation of macrophage colony-stimulating factor production [GO:1901258] Also known as: regulation of M-CSF production Definition: Any process that modulates the frequency, rate or extent of macrophage colony-stimulating factor production. Relationships: is a type of regulation of cytokine production [GO:0001817]; regulates macrophage colony-stimulating factor production [GO:0036301] Sources: GOC:BHF, GOC:TermGenie